{
  "gene_symbol": "ACTL6B",
  "term_id": "GO:0006357",
  "gene": "UniProtKB:O94805",
  "gene_name": "Actin-like protein 6B",
  "term_label": "regulation of transcription by RNA polymerase II"
}